{
  "term_label": "nucleolus",
  "gene": "UniProtKB:Q8NHQ9",
  "gene_symbol": "DDX55",
  "gene_name": "ATP-dependent RNA helicase DDX55",
  "term_id": "GO:0005730"
}